cyclin-dependent protein kinase regulator activity [GO:0019914] (molecular function) Definition: Modulation of the activity of the enzyme cyclin-dependent protein kinase activating kinase. Sources: GOC:ai Relationships: is a type of protein kinase regulator activity [GO:0019887]; regulates cyclin-dependent protein kinase activity [GO:0097472] Subtypes: cyclin-dependent protein serine/threonine kinase regulator activity [GO:0016538] Also known as: cyclin-dependent protein kinase activating kinase, intrinsic regulator activity